{
  "gene_symbol": "BRWD3",
  "term_id": "GO:0005634",
  "term_label": "nucleus",
  "gene_name": "Bromodomain and WD repeat-containing protein 3",
  "gene": "UniProtKB:Q6RI45"
}